{
  "gene_symbol": "TCIRG1",
  "term_label": "proton-transporting ATPase activity, rotational mechanism",
  "term_id": "GO:0046961",
  "gene": "UniProtKB:Q13488",
  "gene_name": "V-type proton ATPase 116 kDa subunit a 3"
}